{
  "gene": "UniProtKB:Q9H5K3",
  "term_id": "GO:0019200",
  "gene_symbol": "POMK",
  "term_label": "carbohydrate kinase activity",
  "gene_name": "Protein O-mannose kinase"
}